{
  "term_label": "Unknown molecular function",
  "term_id": "UNKNOWN:0001",
  "gene_name": "Golgi-associated RAB2 interactor protein 4",
  "gene": "UniProtKB:Q8IYT1",
  "gene_symbol": "GARIN4"
}